guanyl-nucleotide exchange factor complex [GO:0032045] (cellular component) Also known as: guanine nucleotide exchange factor Relationships: is a type of intracellular protein-containing complex [GO:0140535] Subtypes: eukaryotic translation initiation factor 2B complex [GO:0005851], Ric1-Rgp1 guanyl-nucleotide exchange factor complex [GO:0034066], GO:0035658, Ragulator complex [GO:0071986] Sources: GOC:mah Definition: A protein complex that stimulates the exchange of guanyl nucleotides associated with a GTPase.